{
  "gene_name": "Phosphatidylinositide phosphatase SAC2",
  "term_id": "GO:2001135",
  "gene_symbol": "INPP5F",
  "term_label": "regulation of endocytic recycling",
  "gene": "UniProtKB:Q9Y2H2"
}